{
  "gene_symbol": "ZBTB8OS",
  "term_id": "GO:0006388",
  "gene_name": "Protein archease",
  "term_label": "tRNA splicing, via endonucleolytic cleavage and ligation",
  "gene": "UniProtKB:Q8IWT0"
}